regulation of platelet rolling [GO:0160017] (biological process) Relationships: is a type of GO:0034114; regulates GO:0160015 Subtypes: positive regulation of platelet rolling [GO:0160018], negative regulation of platelet rolling [GO:0160019] Definition: Any process that modulates the frequency, rate or extent of platelet rolling. Sources: GOC:sl, GO_REF:0000058